lateral line development [GO:0048882] (biological process) Definition: The process whose specific outcome is the progression of the lateral line over time, from its formation to the mature structure. The lateral line consists of small sensory patches (neuromasts) located superficially on the skin or just under the skin in fluid-filled canals on the head and body of all fishes and most amphibians. The lateral line develops from cranial ectodermal placodes situated behind the ear and between the eye and ear. Also known as: LL development Subtypes: anterior lateral line development [GO:0048899], posterior lateral line development [GO:0048916] Relationships: is a type of tissue development [GO:0009888]; is part of lateral line system development [GO:0048925] Sources: ISBN:0125296509